{
  "term_label": "extracellular space",
  "gene": "UniProtKB:P12259",
  "gene_symbol": "F5",
  "term_id": "GO:0005615",
  "gene_name": "Coagulation factor V"
}